{
  "gene": "UniProtKB:Q5T2T1",
  "term_label": "Unknown molecular function",
  "term_id": "UNKNOWN:0001",
  "gene_name": "MAGUK p55 subfamily member 7",
  "gene_symbol": "MPP7"
}